{
  "gene_symbol": "PCARE",
  "term_id": "GO:0001750",
  "gene": "UniProtKB:A6NGG8",
  "term_label": "photoreceptor outer segment",
  "gene_name": "Photoreceptor cilium actin regulator"
}